ventral aorta morphogenesis [GO:0035913] (biological process) Definition: The process in which the anatomical structures of the ventral aorta are generated and organized. The ventral aorta is a blood vessel in a single-pass circulatory system that carries de-oxygenated blood from the heart to the gills. In a single-pass circulatory system blood passes once through the heart to supply the body once. Sources: GOC:bf, GOC:dgh, UBERON:0003085, Wikipedia:Aorta, ZFA:0000604 Relationships: is a type of aorta morphogenesis [GO:0035909]; is part of GO:0035908